{
  "term_label": "extracellular matrix organization",
  "term_id": "GO:0030198",
  "gene_name": "Vitrin",
  "gene_symbol": "VIT",
  "gene": "UniProtKB:Q6UXI7"
}